{
  "gene_symbol": "SYTL2",
  "term_id": "GO:0042043",
  "gene_name": "Synaptotagmin-like protein 2",
  "gene": "UniProtKB:Q9HCH5",
  "term_label": "neurexin family protein binding"
}